{
  "term_label": "G1/S transition of mitotic cell cycle",
  "gene": "UniProtKB:Q9NRM7",
  "gene_symbol": "LATS2",
  "gene_name": "Serine_threonine-protein kinase LATS2",
  "term_id": "GO:0000082"
}